{
  "term_id": "GO:0005925",
  "gene_name": "Protein-tyrosine kinase 2-beta",
  "term_label": "focal adhesion",
  "gene": "UniProtKB:Q14289",
  "gene_symbol": "PTK2B"
}